{
  "gene_name": "C3a anaphylatoxin chemotactic receptor",
  "term_id": "GO:0004930",
  "gene": "UniProtKB:Q16581",
  "term_label": "G protein-coupled receptor activity",
  "gene_symbol": "C3AR1"
}